{
  "gene_name": "Coiled-coil domain-containing protein 105",
  "term_id": "UNKNOWN:0002",
  "gene": "UniProtKB:Q8IYK2",
  "term_label": "Unknown biological process",
  "gene_symbol": "CCDC105"
}